{
  "gene": "UniProtKB:Q9NNW7",
  "term_id": "GO:0005739",
  "gene_name": "Thioredoxin reductase 2, mitochondrial",
  "gene_symbol": "TXNRD2",
  "term_label": "mitochondrion"
}